response to interleukin-4 [GO:0070670] (biological process) Also known as: response to IL-4 Subtypes: GO:0071353 Relationships: is a type of response to cytokine [GO:0034097] Sources: GOC:mah Definition: Any process that results in a change in state or activity of a cell or an organism (in terms of movement, secretion, enzyme production, gene expression, etc.) as a result of an interleukin-4 stimulus.